{
  "gene_name": "Serine_threonine-protein kinase ULK2",
  "term_id": "GO:0034727",
  "gene": "UniProtKB:Q8IYT8",
  "gene_symbol": "ULK2",
  "term_label": "piecemeal microautophagy of the nucleus"
}